R2/R5 development [GO:0048055] (biological process) Sources: GOC:jid Definition: The process whose specific outcome is the progression of the R2 and R5 pair of photoreceptors in the eye over time, from their formation to the mature structures. R2 and R5 are paired photoreceptors that contribute to the outer rhabdomeres. An example of this process is found in Drosophila melanogaster. Relationships: is a type of compound eye photoreceptor development [GO:0042051]; is part of R2/R5 cell differentiation [GO:0048054]